{
  "gene_symbol": "CHMP5",
  "gene_name": "Charged multivesicular body protein 5",
  "term_id": "GO:0005771",
  "term_label": "multivesicular body",
  "gene": "UniProtKB:Q9NZZ3"
}